regulation of central B cell tolerance induction [GO:0002895] (biological process) Subtypes: GO:0002896, positive regulation of central B cell tolerance induction [GO:0002897], GO:0002898, regulation of central B cell anergy [GO:0002914] Relationships: is a type of regulation of central tolerance induction [GO:0002646]; is a type of regulation of B cell tolerance induction [GO:0002661]; RO_0002211 GO:0002510 Sources: GOC:add Definition: Any process that modulates the frequency, rate, or extent of central B cell tolerance induction.